{
  "gene_name": "DNA-directed RNA polymerase III subunit RPC7",
  "term_id": "UNKNOWN:0001",
  "gene": "UniProtKB:O15318",
  "term_label": "Unknown molecular function",
  "gene_symbol": "POLR3G"
}